{
  "gene_name": "Testis-expressed protein 35",
  "gene": "UniProtKB:Q5T0J7",
  "gene_symbol": "TEX35",
  "term_id": "GO:0005634",
  "term_label": "nucleus"
}